microtubule cytoskeleton organization [GO:0000226] (biological process) Sources: GOC:mah Definition: A process that is carried out at the cellular level which results in the assembly, arrangement of constituent parts, or disassembly of cytoskeletal structures comprising microtubules and their associated proteins. Subtypes: microtubule bundle formation [GO:0001578], microtubule nucleation [GO:0007020], spindle organization [GO:0007051], radial microtubular system formation [GO:0010245], modulation of microtubule cytoskeleton involved in cerebral cortex radial glia guided migration [GO:0021815], establishment or maintenance of microtubule cytoskeleton polarity [GO:0030951], microtubule polymerization or depolymerization [GO:0031109], GO:0031121, GO:0031122, horsetail-astral microtubule organization [GO:0032118], microtubule anchoring [GO:0034453], sperm aster formation [GO:0035044], microtubule severing [GO:0051013], GO:0051293, phragmoplast microtubule organization [GO:0080175], microtubule cytoskeleton organization involved in establishment of planar polarity [GO:0090176], GO:1902850, microtubule cytoskeleton attachment to nuclear envelope [GO:1990933] Also known as: microtubule cytoskeleton organisation, microtubule cytoskeleton organization and biogenesis Relationships: is a type of GO:0007010; is_a microtubule-based process [GO:0007017] Regulation: regulated by regulation of microtubule cytoskeleton organization [GO:0070507]